cardiac neural crest cell migration involved in outflow tract morphogenesis [GO:0003253] (biological process) Definition: The orderly movement of a neural crest cell from one site to another that will contribute to the morphogenesis of the outflow tract. Sources: GOC:mtg_heart Regulation: regulated by GO:1905310; negatively regulated by GO:1905311; positively regulated by GO:1905312 Relationships: is a type of neural crest cell migration [GO:0001755]; is a type of cell migration involved in heart development [GO:0060973]; is part of cardiac neural crest cell development involved in outflow tract morphogenesis [GO:0061309]